positive regulation of silent mating-type cassette heterochromatin formation [GO:0090055] (biological process) Definition: Any process that increases the frequency, rate, or extent of heterochromatin formation at silent mating-type cassette. Sources: GOC:dph, GOC:tb Relationships: is a type of positive regulation of heterochromatin formation [GO:0031453]; is a type of regulation of silent mating-type cassette heterochromatin formation [GO:0090054]; RO_0002213 silent mating-type cassette heterochromatin formation [GO:0030466] Also known as: positive regulation of chromatin silencing at silent mating-type cassette, positive regulation of silent mating-type cassette heterochromatin assembly